{
  "gene": "UniProtKB:O14662",
  "term_id": "GO:0031201",
  "term_label": "SNARE complex",
  "gene_name": "Syntaxin-16",
  "gene_symbol": "STX16"
}